{
  "gene_symbol": "C11orf16",
  "gene_name": "Uncharacterized protein C11orf16",
  "gene": "UniProtKB:Q9NQ32",
  "term_id": "UNKNOWN:0001",
  "term_label": "Unknown molecular function"
}